{
  "term_id": "GO:0016925",
  "term_label": "protein sumoylation",
  "gene": "UniProtKB:O75925",
  "gene_name": "E3 SUMO-protein ligase PIAS1",
  "gene_symbol": "PIAS1"
}